{
  "gene_symbol": "DBF4B",
  "gene_name": "Protein DBF4 homolog B",
  "term_id": "GO:1901987",
  "term_label": "regulation of cell cycle phase transition",
  "gene": "UniProtKB:Q8NFT6"
}